protein kinase A binding [GO:0051018] (molecular function) Also known as: PKA binding, protein kinase A anchoring activity Note: Note that this term is a direct child of 'protein binding ; GO:0005515' because it encompasses binding to either the catalytic or regulatory subunit of protein kinase A, and the latter does not have kinase activity. Definition: Binding to a protein kinase A. Sources: GOC:ai Subtypes: GO:0034236, GO:0034237 Relationships: is a type of protein binding [GO:0005515]